negative regulation of T-helper 17 cell differentiation [GO:2000320] (biological process) Relationships: is_a negative regulation of T-helper cell differentiation [GO:0045623]; is a type of GO:2000317; is a type of regulation of T-helper 17 cell differentiation [GO:2000319]; negatively regulates T-helper 17 cell differentiation [GO:0072539] Subtypes: negative regulation of T-helper 17 cell lineage commitment [GO:2000329] Definition: Any process that stops, prevents or reduces the frequency, rate or extent of T-helper 17 cell differentiation. Sources: GOC:BHF, GOC:mah Also known as: negative regulation of T-helper 17 cell development